{
  "gene_name": "Tyrosine-protein kinase ITK_TSK",
  "term_label": "adaptive immune response",
  "gene": "UniProtKB:Q08881",
  "term_id": "GO:0002250",
  "gene_symbol": "ITK"
}